sulfur oxygenase/reductase activity [GO:0033755] (molecular function) Definition: Catalysis of the reaction: 4 sulfur + 4 H2O + O2 = 2 hydrogen sulfide + 2 bisulfite + 2 H+. References: PMID:1522063 Sources: EC:1.13.11.55 Also known as: sulfur oxygenase activity, sulphur oxygenase/reductase activity, SOR, sulfur:oxygen oxidoreductase (hydrogen-sulfide- and sulfite-forming) activity Relationships: is a type of GO:0016702